{
  "term_label": "regulation of small GTPase mediated signal transduction",
  "gene_name": "Rho GTPase-activating protein 40",
  "gene": "UniProtKB:Q5TG30",
  "term_id": "GO:0051056",
  "gene_symbol": "ARHGAP40"
}